Rad17 RFC-like complex [GO:0031389] (cellular component) Relationships: is a type of protein-containing complex [GO:0032991]; is part of chromosome [GO:0005694] Definition: A pentameric protein complex related to replication factor C, which loads a trimeric complex of checkpoint proteins (known as the checkpoint clamp or 9-1-1 complex) onto DNA at damage sites; functions in DNA damage cell cycle checkpoints. In Schizosaccharomyces pombe the subunits are known as Rad17, Rfc2, Rfc3, Rfc4, and Rfc5, while in Saccharomyces cerevisiae the subunits are known as Rad24p, Rfc2p, Rfc3p, Rfc4p, and Rfc5p. Also known as: RFC (Rad17), Rad17-RFC, Rad17-RLC, Rad24p RFC-like complex References: PMID:14614842